{
  "term_id": "UNKNOWN:0001",
  "gene_name": "Low-density lipoprotein receptor-related protein 11",
  "gene": "UniProtKB:Q86VZ4",
  "term_label": "Unknown molecular function",
  "gene_symbol": "LRP11"
}